{
  "term_id": "UNKNOWN:0003",
  "gene_symbol": "IKZF4",
  "term_label": "Unknown cellular component",
  "gene_name": "Zinc finger protein Eos",
  "gene": "UniProtKB:Q9H2S9"
}